bicarbonate channel activity [GO:0160133] (molecular function) Definition: Enables the energy-independent facilitated diffusion of bicarbonate through a transmembrane aqueous pore or channel. References: PMID:18400985 Also known as: hydrogencarbonate channel activity Relationships: is a type of bicarbonate transmembrane transporter activity [GO:0015106]; is a type of GO:0015267